malonate CoA-transferase activity [GO:0050078] (molecular function) Definition: Catalysis of the reaction: acetyl-CoA + malonate = acetate + malonyl-CoA. Sources: EC:2.8.3.3, RHEA:18817 Also known as: acetyl-CoA:malonate CoA-transferase activity, malonate coenzyme A-transferase activity Relationships: is a type of CoA-transferase activity [GO:0008410]